{
  "term_id": "UNKNOWN:0002",
  "gene_name": "C1GALT1-specific chaperone 1",
  "gene_symbol": "C1GALT1C1",
  "gene": "UniProtKB:Q96EU7",
  "term_label": "Unknown biological process"
}